{
  "term_label": "cytoplasm",
  "gene_name": "Enhancer of filamentation 1",
  "gene_symbol": "NEDD9",
  "gene": "UniProtKB:Q14511",
  "term_id": "GO:0005737"
}